{
  "gene": "UniProtKB:Q96JM2",
  "gene_name": "Zinc finger protein 462",
  "term_id": "GO:0006355",
  "term_label": "regulation of DNA-templated transcription",
  "gene_symbol": "ZNF462"
}